{
  "gene_name": "Beta-crystallin B3",
  "term_label": "lens development in camera-type eye",
  "term_id": "GO:0002088",
  "gene_symbol": "CRYBB3",
  "gene": "UniProtKB:P26998"
}